{
  "gene": "UniProtKB:Q7RTT4",
  "term_label": "Unknown biological process",
  "gene_symbol": "SSX8P",
  "gene_name": "Putative protein SSX8",
  "term_id": "UNKNOWN:0002"
}